microsporidian-type exospore [GO:0090642] (CC) Relationships: is_a GO:0110165; is part of spore wall [GO:0031160] Definition: The dense, protein rich outermost layer of a microsporidian spore wall that lies above the endospore. References: PMID:19457051, PMID:25363531